{
  "term_label": "guanyl-nucleotide exchange factor activity",
  "term_id": "GO:0005085",
  "gene_name": "Cytohesin-1",
  "gene": "UniProtKB:Q15438",
  "gene_symbol": "CYTH1"
}